{
  "term_label": "Unknown biological process",
  "gene_name": "Ubiquitin domain-containing protein UBFD1",
  "term_id": "UNKNOWN:0002",
  "gene_symbol": "UBFD1",
  "gene": "UniProtKB:O14562"
}